medium-chain fatty acid omega-hydroxylase activity [GO:0140981] (molecular function) Relationships: is a type of fatty acid omega-hydroxylase activity [GO:0120250] Sources: RHEA:75279 Definition: Catalysis of the reaction: an omega-methyl-medium-chain fatty acid + O2 + reduced [NADPH--hemoprotein reductase] = an omega-hydroxy-medium-chain fatty acid + H+ + H2O + oxidized [NADPH--hemoprotein reductase]. A medium-chain fatty acid has an aliphatic tail containing 6 to 12 carbons. Note: While there is not universal consensus on the lengths of short-, medium-, long- and very-long-chain fatty acids, the GO uses the definitions in ChEBI (see CHEBI:26666, CHEBI:59554, CHEBI:15904 and CHEBI:27283).